{
  "term_id": "GO:0090090",
  "term_label": "negative regulation of canonical Wnt signaling pathway",
  "gene_name": "Adenomatous polyposis coli protein",
  "gene_symbol": "APC",
  "gene": "UniProtKB:P25054"
}